{
  "gene_symbol": "PRPF18",
  "gene": "UniProtKB:Q99633",
  "gene_name": "Pre-mRNA-splicing factor 18",
  "term_id": "GO:0071021",
  "term_label": "U2-type post-spliceosomal complex"
}